{
  "term_label": "cytoplasm",
  "gene_symbol": "EIF1AX",
  "term_id": "GO:0005737",
  "gene": "UniProtKB:P47813",
  "gene_name": "Eukaryotic translation initiation factor 1A, X-chromosomal"
}